interferon-alpha production [GO:0032607] (biological process) Regulation: regulated by regulation of interferon-alpha production [GO:0032647]; negatively regulated by negative regulation of interferon-alpha production [GO:0032687]; RO_0002213 by positive regulation of interferon-alpha production [GO:0032727] Also known as: IFN-alpha production, IFNA production, interferon-alpha biosynthetic process, interferon-alpha secretion Note: Note that this term is in the subset of terms that should not be used for direct gene product annotation. Instead, select one of the 'regulation' children terms. Relationships: is_a type I interferon production [GO:0032606] Definition: The appearance of interferon-alpha due to biosynthesis or secretion following a cellular stimulus, resulting in an increase in its intracellular or extracellular levels. References: PMID:15546383 Sources: GOC:mah